{
  "gene": "UniProtKB:A6NI61",
  "term_id": "GO:0007520",
  "term_label": "myoblast fusion",
  "gene_symbol": "MYMK",
  "gene_name": "Protein myomaker"
}